cellobiose binding [GO:0044585] (molecular function) Definition: Binding to cellobiose, a disaccharide that represents the basic repeating unit of cellulose. Relationships: is a type of disaccharide binding [GO:0048030] Sources: GOC:mengo_curators, GOC:tt